host cell endoplasmic reticulum lumen [GO:0044166] (CC) Definition: The volume enclosed by the membranes of the host cell endoplasmic reticulum. Relationships: is a type of GO:0033655; is part of host cell endoplasmic reticulum [GO:0044165] Sources: GOC:jl Also known as: host endoplasmic reticulum lumen